{
  "term_label": "late endosome membrane",
  "term_id": "GO:0031902",
  "gene_symbol": "HLA-DQA1",
  "gene": "UniProtKB:P01909",
  "gene_name": "HLA class II histocompatibility antigen, DQ alpha 1 chain"
}